corticospinal tract morphogenesis [GO:0021957] (biological process) Definition: Generation of a long process of a pyramidal cell, that carries efferent (outgoing) action potentials from the cell body in cerebral cortex layer V towards target cells in the gray matter of the spinal cord. This axonal process is a member of those that make up the corticospinal tract. Relationships: is a type of central nervous system projection neuron axonogenesis [GO:0021952] References: PMID:9878731 Sources: GOC:cls, GOC:dgh, GOC:dph, GOC:jid, GO_REF:0000021 Also known as: CST axonogenesis, corticospinal tract axonogenesis